{
  "term_label": "Unknown cellular component",
  "gene_name": "Putative cytochrome P450 family member 4F30",
  "gene": "UniProtKB:Q9H0H9",
  "gene_symbol": "CYP4F30P",
  "term_id": "UNKNOWN:0003"
}